{
  "gene_name": "Cell division cycle protein 27 homolog",
  "gene": "UniProtKB:P30260",
  "gene_symbol": "CDC27",
  "term_label": "anaphase-promoting complex",
  "term_id": "GO:0005680"
}